ryanodine-sensitive calcium-release channel activity [GO:0005219] (molecular function) Subtypes: ryanodine-sensitive calcium-release channel activity involved in regulation of postsynaptic cytosolic calcium levels [GO:0098697] Also known as: ryanodine receptor, caffeine-sensitive calcium-release channel Regulation: regulated by regulation of ryanodine-sensitive calcium-release channel activity [GO:0060314]; negatively regulated by GO:0060315 References: PMID:22822064 Sources: GOC:dph, GOC:tb Relationships: is a type of calcium-induced calcium release activity [GO:0048763] Definition: Enables transmembrane transfer of calcium ions from an intracellular store to the cytosol on induction by increased calcium concentration and is sensitive to the plant alkaloid ryanodine.